{
  "gene": "UniProtKB:O75783",
  "term_label": "Unknown biological process",
  "term_id": "UNKNOWN:0002",
  "gene_symbol": "RHBDL1",
  "gene_name": "Rhomboid-related protein 1"
}